{
  "gene_name": "L-xylulose reductase",
  "gene": "UniProtKB:Q7Z4W1",
  "gene_symbol": "DCXR",
  "term_id": "GO:0004090",
  "term_label": "carbonyl reductase (NADPH) activity"
}